{
  "gene_name": "Olfactory receptor 51B6",
  "term_id": "GO:0005886",
  "gene_symbol": "OR51B6",
  "gene": "UniProtKB:Q9H340",
  "term_label": "plasma membrane"
}